{
  "gene_symbol": "OSMR",
  "term_id": "GO:0009897",
  "gene": "UniProtKB:Q99650",
  "term_label": "external side of plasma membrane",
  "gene_name": "Oncostatin-M-specific receptor subunit beta"
}